potassium ion leak channel activity [GO:0022841] (MF) Relationships: is a type of potassium channel activity [GO:0005267]; is a type of leak channel activity [GO:0022840] Definition: Enables the transport of a potassium ion across a membrane via a narrow pore channel that is open even in an unstimulated or 'resting' state. Sources: GOC:mtg_transport, ISBN:0815340729